{
  "gene_symbol": "NPIPA9",
  "gene_name": "Nuclear pore complex-interacting protein family member A9",
  "term_id": "UNKNOWN:0002",
  "gene": "UniProtKB:A0A0B4J1W7",
  "term_label": "Unknown biological process"
}